{
  "term_id": "GO:0006911",
  "term_label": "phagocytosis, engulfment",
  "gene": "UniProtKB:Q9UBW5",
  "gene_name": "Bridging integrator 2",
  "gene_symbol": "BIN2"
}